positive regulation of intestinal epithelial cell development [GO:1905300] (biological process) Relationships: is a type of positive regulation of cell development [GO:0010720]; is a type of positive regulation of multicellular organismal process [GO:0051240]; is a type of regulation of intestinal epithelial cell development [GO:1905298]; positively regulates intestinal epithelial cell development [GO:0060576] References: PMID:23904268 Sources: GOC:BHF, GOC:BHF_miRNA, GOC:TermGenie, GOC:rph, GO_REF:0000058 Also known as: up regulation of intestinal epithelial cell development, up-regulation of intestinal epithelial cell development, upregulation of intestinal epithelial cell development, activation of intestinal epithelial cell development Definition: Any process that activates or increases the frequency, rate or extent of intestinal epithelial cell development.